{
  "gene_symbol": "LSM5",
  "term_label": "U4/U6 x U5 tri-snRNP complex",
  "gene_name": "U6 snRNA-associated Sm-like protein LSm5",
  "gene": "UniProtKB:Q9Y4Y9",
  "term_id": "GO:0046540"
}